{
  "gene_name": "Immunoglobulin heavy variable 3-49",
  "term_id": "UNKNOWN:0003",
  "gene": "UniProtKB:A0A0A0MS15",
  "gene_symbol": "IGHV3-49",
  "term_label": "Unknown cellular component"
}